{
  "term_label": "immune response",
  "gene_symbol": "IGKV1D-42",
  "gene": "UniProtKB:A0A075B6H8",
  "gene_name": "Probable non-functional immunoglobulin kappa variable 1D-42",
  "term_id": "GO:0006955"
}